{
  "term_id": "UNKNOWN:0001",
  "gene": "UniProtKB:Q9UL63",
  "term_label": "Unknown molecular function",
  "gene_name": "Muskelin",
  "gene_symbol": "MKLN1"
}